{
  "gene_symbol": "SOWAHC",
  "term_id": "UNKNOWN:0002",
  "term_label": "Unknown biological process",
  "gene": "UniProtKB:Q53LP3",
  "gene_name": "Ankyrin repeat domain-containing protein SOWAHC"
}